protoporphyrinogen oxidase activity [GO:0070818] (molecular function) Definition: Catalysis of the reaction: protoporphyrinogen IX + acceptor = protoporphyrin IX + reduced acceptor. References: PMID:19583219 Sources: GOC:mah Also known as: protoporphyrinogen IX oxidase activity, protoporphyrinogen-IX oxidase activity, protoporphyrinogenase activity Relationships: is a type of GO:0016627 Subtypes: oxygen-dependent protoporphyrinogen oxidase activity [GO:0004729], menaquinone-dependent protoporphyrinogen oxidase activity [GO:0070819]